{
  "gene_name": "Tetratricopeptide repeat protein 36",
  "term_id": "UNKNOWN:0001",
  "term_label": "Unknown molecular function",
  "gene": "UniProtKB:A6NLP5",
  "gene_symbol": "TTC36"
}